basolateral protein secretion [GO:0110010] (biological process) References: PMID:27404358 Sources: GOC:ha Definition: The controlled release of proteins from a cell at the sides which interface adjacent cells and near the base. Relationships: is a type of protein secretion [GO:0009306]